{
  "term_label": "poly(A)+ mRNA export from nucleus",
  "term_id": "GO:0016973",
  "gene_name": "ATP-dependent RNA helicase DDX19A",
  "gene_symbol": "DDX19A",
  "gene": "UniProtKB:Q9NUU7"
}